glycolytic process via Entner-Doudoroff Pathway [GO:0061688] (biological process) References: PMID:9657988 Sources: GOC:dph Also known as: gluconate pathway Relationships: is_a GO:0006096; has part Entner-Doudoroff pathway [GO:0061678] Definition: A glycolytic process in which the glucose is catabolized to pyruvate by first entering the Entner-Doudoroff pathway to yield pyruvate and glyceraldehyde-3-phosphate. The glyceraldehyde-3-phosphate is subsequently converted to pyruvate by the core glycolytic enzymes.